{
  "gene_symbol": "PRAMEF11",
  "term_label": "ubiquitin-like ligase-substrate adaptor activity",
  "gene_name": "PRAME family member 11",
  "gene": "UniProtKB:O60813",
  "term_id": "GO:1990756"
}